{
  "gene": "UniProtKB:Q9UN81",
  "gene_symbol": "L1RE1",
  "gene_name": "LINE-1 retrotransposable element ORF1 protein",
  "term_label": "retrotransposition",
  "term_id": "GO:0032197"
}